glycine hydroxymethyltransferase activity [GO:0004372] (molecular function) Also known as: 5,10-methylenetetrahydrofolate:glycine hydroxymethyltransferase activity, L-serine hydroxymethyltransferase activity, allothreonine aldolase activity, serine aldolase activity, serine hydroxymethylase activity, serine hydroxymethyltransferase activity, serine transhydroxymethylase activity Definition: Catalysis of the reaction: (6R)-5,10-methylene-5,6,7,8-tetrahydrofolate + glycine + H2O = (6S)-5,6,7,8-tetrahydrofolate + L-serine. Sources: RHEA:15481 Relationships: is a type of hydroxymethyl-, formyl- and related transferase activity [GO:0016742]